{
  "gene_symbol": "ORMDL2",
  "term_id": "GO:0006672",
  "gene": "UniProtKB:Q53FV1",
  "term_label": "ceramide metabolic process",
  "gene_name": "ORM1-like protein 2"
}